sulfate adenylyltransferase (ATP) activity [GO:0004781] (molecular function) Definition: Catalysis of the reaction: ATP + H+ + sulfate = adenosine 5'-phosphosulfate + diphosphate. Also known as: ATP:sulfate adenylyltransferase activity, sulphate adenylyltransferase (ATP) activity, ATP sulfurylase activity, ATP-sulfurylase activity, adenosine-5'-triphosphate sulfurylase activity, adenosinetriphosphate sulfurylase activity, adenylylsulfate pyrophosphorylase activity, sulfate adenylate transferase activity, sulfurylase activity Relationships: is a type of GO:0004779 Sources: EC:2.7.7.4